group A colicin transmembrane transporter activity [GO:0042913] (molecular function) Relationships: is a type of colicin transmembrane transporter activity [GO:0042912] References: PMID:9171417 Sources: GOC:jl, GOC:mtg_transport, ISBN:0815340729 Definition: Enables the transfer of group A colicins (colicins E1, E2, E3, A, K, and N) from one side of a membrane to the other.